COPI-coated vesicle lumen [GO:0106172] (cellular component) Definition: The volume enclosed by the membrane of a COPI-coated endocytic vesicle. References: PMID:29535154 Sources: GOC:pde Relationships: is a type of cytoplasmic vesicle lumen [GO:0060205]; BFO_0000050 COPI-coated vesicle [GO:0030137]